mesenchymal cell fate commitment [GO:0014030] (biological process) Relationships: is a type of cell fate commitment [GO:0045165]; is part of mesenchymal cell differentiation [GO:0048762] Definition: The process in which a cell becomes committed to become a mesenchymal cell. Sources: GOC:dh, GOC:ef